{
  "gene_name": "Homeodomain-interacting protein kinase 3",
  "gene_symbol": "HIPK3",
  "gene": "UniProtKB:Q9H422",
  "term_id": "GO:0005634",
  "term_label": "nucleus"
}